{
  "gene_name": "All-trans retinoic acid-induced differentiation factor",
  "term_label": "positive regulation of osteoblast differentiation",
  "gene": "UniProtKB:Q6UW56",
  "gene_symbol": "ATRAID",
  "term_id": "GO:0045669"
}